{
  "term_label": "antimicrobial humoral immune response mediated by antimicrobial peptide",
  "gene_symbol": "CCL18",
  "gene_name": "C-C motif chemokine 18",
  "gene": "UniProtKB:P55774",
  "term_id": "GO:0061844"
}